cellular response to triterpenoid [GO:1905837] (biological process) Relationships: is a type of cellular response to lipid [GO:0071396]; is a type of response to triterpenoid [GO:1905836] Subtypes: cellular response to diosgenin [GO:1905093] References: PMID:28078994 Sources: GOC:TermGenie, GO_REF:0000071 Definition: Any process that results in a change in state or activity of a cell (in terms of movement, secretion, enzyme production, gene expression, etc.) as a result of a triterpenoid stimulus.